{
  "term_id": "GO:0005634",
  "term_label": "nucleus",
  "gene_name": "Nuclear receptor coactivator 7",
  "gene": "UniProtKB:Q8NI08",
  "gene_symbol": "NCOA7"
}